{
  "term_label": "protein tyrosine phosphatase activity",
  "gene_symbol": "PTPRG",
  "gene_name": "Receptor-type tyrosine-protein phosphatase gamma",
  "term_id": "GO:0004725",
  "gene": "UniProtKB:P23470"
}